{
  "term_id": "GO:1901888",
  "gene_symbol": "ROCK1",
  "term_label": "regulation of cell junction assembly",
  "gene": "UniProtKB:Q13464",
  "gene_name": "Rho-associated protein kinase 1"
}